{
  "term_label": "Unknown molecular function",
  "gene_symbol": "CFAP20",
  "gene": "UniProtKB:Q9Y6A4",
  "gene_name": "Cilia- and flagella-associated protein 20",
  "term_id": "UNKNOWN:0001"
}